{
  "gene_name": "U3 small nucleolar RNA-associated protein 14 homolog A",
  "term_id": "UNKNOWN:0002",
  "gene_symbol": "UTP14A",
  "term_label": "Unknown biological process",
  "gene": "UniProtKB:Q9BVJ6"
}